{
  "gene": "UniProtKB:P02647",
  "term_label": "cholesterol efflux",
  "gene_name": "Apolipoprotein A-I",
  "gene_symbol": "APOA1",
  "term_id": "GO:0033344"
}